{
  "gene_name": "Negative elongation factor B",
  "term_label": "negative regulation of transcription elongation by RNA polymerase II",
  "gene": "UniProtKB:Q8WX92",
  "gene_symbol": "NELFB",
  "term_id": "GO:0034244"
}